{
  "gene_symbol": "RNF114",
  "term_label": "ubiquitin-dependent protein catabolic process",
  "term_id": "GO:0006511",
  "gene_name": "E3 ubiquitin-protein ligase RNF114",
  "gene": "UniProtKB:Q9Y508"
}